endoplasmic reticulum cisternal network organization [GO:0071783] (biological process) Also known as: ER cisternal network organisation, ER cisternal network organization, endoplasmic reticulum cisternal network organisation References: PMID:16469703, PMID:20434336 Sources: GOC:vw Definition: A process that is carried out at the cellular level which results in the assembly, arrangement of constituent parts, or disassembly of the endoplasmic reticulum (ER) cisternal network. The ER cisternal network is the ER part that comprises the membranes with low curvature in cross-section. Subtypes: endoplasmic reticulum cisternal network assembly [GO:0071784], endoplasmic reticulum cisternal network maintenance [GO:0071785] Relationships: is a type of endoplasmic reticulum organization [GO:0007029]